accessory nerve structural organization [GO:0021609] (biological process) Also known as: accessory nerve structural organisation, CN XI structural organization Sources: GOC:cls, GOC:dgh, GOC:dph, GOC:jid, GO_REF:0000021 Relationships: is a type of GO:0021604; is part of accessory nerve morphogenesis [GO:0021607] Definition: The process that contributes to the act of creating the structural organization of the accessory nerve This process pertains to the physical shaping of a rudimentary structure. The spinal branch of this motor nerve innervates the trapezius and the sternocleidomastoid muscles. The cranial branch joins the vagus nerve and innervates the same targets as the vagus nerve.